{
  "gene_symbol": "ATP1A3",
  "gene_name": "Sodium_potassium-transporting ATPase subunit alpha-3",
  "term_label": "proton transmembrane transport",
  "gene": "UniProtKB:P13637",
  "term_id": "GO:1902600"
}